{
  "gene_symbol": "CCDC169",
  "gene": "UniProtKB:A6NNP5",
  "term_label": "Unknown biological process",
  "term_id": "UNKNOWN:0002",
  "gene_name": "Coiled-coil domain-containing protein 169"
}